{
  "term_id": "GO:0006302",
  "gene_name": "182 kDa tankyrase-1-binding protein",
  "gene": "UniProtKB:Q9C0C2",
  "term_label": "double-strand break repair",
  "gene_symbol": "TNKS1BP1"
}